intramolecular oxidoreductase activity, transposing S-S bonds [GO:0016864] (molecular function) Subtypes: protein disulfide isomerase activity [GO:0003756] Also known as: intramolecular isomerase activity, transposing S-S bonds Definition: Catalysis of an oxidation-reduction (redox) reaction in which the hydrogen donor and acceptor are the same molecule, one or more sulfur-sulfur bonds in the molecule are rearranged, and no oxidized product appears. Sources: EC:5.3.4.-, GOC:mah Relationships: is a type of GO:0016860